{
  "gene_name": "Urocortin-2",
  "term_id": "GO:0051429",
  "gene": "UniProtKB:Q96RP3",
  "gene_symbol": "UCN2",
  "term_label": "corticotropin-releasing hormone receptor binding"
}